metal incorporation into metallo-sulfur cluster [GO:0018282] (biological process) Definition: The formation of a cluster of several metal atoms, including iron, nickel, molybdenum, vanadium, or copper, with one or more bridging (mu-bond) sulfur atoms; amino acids residues in proteins that may ligate the metal sulfur cluster are cysteine, histidine, aspartate, glutamate, serine and cysteine persulfide. Sources: GOC:jsg Also known as: metal incorporation into metallo-sulphur cluster Relationships: is a type of GO:0036211; is part of metallo-sulfur cluster assembly [GO:0031163] Subtypes: iron incorporation into metallo-sulfur cluster [GO:0018283], molybdenum incorporation into metallo-sulfur cluster [GO:0018289], nickel incorporation into metallo-sulfur cluster [GO:0018414], copper incorporation into metallo-sulfur cluster [GO:0018427]